(S)-scoulerine biosynthetic process [GO:1901009] (biological process) Definition: The chemical reactions and pathways resulting in the formation of (S)-scoulerine. Relationships: is a type of isoquinoline alkaloid biosynthetic process [GO:0033075] Also known as: (S)-scoulerine anabolism, (S)-scoulerine biosynthesis, (S)-scoulerine formation, (S)-scoulerine synthesis References: PMID:15672841 Sources: GOC:TermGenie, GOC:yaf